B cell receptor transport within lipid bilayer [GO:0032595] (biological process) Definition: The directed movement of a B cell receptor within a lipid bilayer. Also known as: B cell receptor translocation within membrane, BCR translocation within membrane, BCR transport within lipid bilayer Sources: GOC:mah Relationships: is a type of protein transport within lipid bilayer [GO:0032594] Subtypes: GO:0032597